{
  "gene_name": "Glutamate receptor 2",
  "gene_symbol": "GRIA2",
  "term_id": "GO:0005886",
  "gene": "UniProtKB:P42262",
  "term_label": "plasma membrane"
}